positive regulation of Rho protein signal transduction [GO:0035025] (biological process) Relationships: is_a regulation of Rho protein signal transduction [GO:0035023]; is a type of GO:0051057; positively regulates GO:0007266 Also known as: up regulation of Rho protein signal transduction, up-regulation of Rho protein signal transduction, upregulation of Rho protein signal transduction, activation of Rho protein signal transduction, stimulation of Rho protein signal transduction Sources: GOC:bf Definition: Any process that activates or increases the frequency, rate or extent of Rho protein signal transduction.